{
  "gene_name": "Transmembrane protein 191C",
  "term_label": "Unknown cellular component",
  "gene_symbol": "TMEM191C",
  "term_id": "UNKNOWN:0003",
  "gene": "UniProtKB:A6NGB0"
}